aminobenzoate decarboxylase activity [GO:0047662] (molecular function) Also known as: aminobenzoate carboxy-lyase (aniline-forming), aminobenzoate carboxy-lyase activity Sources: EC:4.1.1.24, MetaCyc:AMINOBENZOATE-DECARBOXYLASE-RXN Definition: Catalysis of the reaction: 4(or 2)-aminobenzoate = aniline + CO2. Relationships: is a type of carboxy-lyase activity [GO:0016831]